extracellular exosome assembly [GO:0071971] (biological process) Relationships: is a type of GO:0016050; is a type of organelle assembly [GO:0070925]; is part of extracellular exosome biogenesis [GO:0097734] Regulation: regulated by GO:1903551; negatively regulated by negative regulation of extracellular exosome assembly [GO:1903552]; RO_0002213 by positive regulation of extracellular exosome assembly [GO:1903553] Also known as: extracellular vesicular exosome assembly Definition: The aggregation, arrangement and bonding together of a set of components to form an extracellular vesicular exosome, a membrane-bounded vesicle that is released into the extracellular region by fusion of the limiting endosomal membrane of a multivesicular body with the plasma membrane. Exosomes are defined by their size, which generally ranges from 30 nm to 100 nm. References: PMID:19442504, PMID:27462458 Sources: GOC:mah, GOC:tfm